{
  "gene_name": "Diacylglycerol kinase delta",
  "term_id": "GO:0005886",
  "term_label": "plasma membrane",
  "gene_symbol": "DGKD",
  "gene": "UniProtKB:Q16760"
}